{
  "term_label": "Unknown molecular function",
  "gene_symbol": "CATR1",
  "gene": "UniProtKB:Q13166",
  "gene_name": "CATR tumorigenic conversion 1 protein",
  "term_id": "UNKNOWN:0001"
}